brain-derived neurotrophic factor binding [GO:0048403] (molecular function) Definition: Binding to brain-derived neurotrophic factor. Sources: GOC:dgh Also known as: BDNF binding, neurotrophin TRKB receptor activity Relationships: is a type of GO:0043121